UDP-D-galacturonate biosynthetic process [GO:0033480] (biological process) Definition: The chemical reactions and pathways resulting in the formation of UDP-D-galacturonate, a substance composed of galacturonic acid in glycosidic linkage with uridine diphosphate. Sources: GOC:mah Also known as: UDP-D-galacturonate anabolism, UDP-D-galacturonate biosynthesis, UDP-D-galacturonate formation, UDP-D-galacturonate synthesis Relationships: is a type of nucleotide-sugar biosynthetic process [GO:0009226]